{
  "term_label": "protein folding chaperone",
  "gene_symbol": "LYRM7",
  "gene_name": "Complex III assembly factor LYRM7",
  "gene": "UniProtKB:Q5U5X0",
  "term_id": "GO:0044183"
}